{
  "term_id": "GO:0005768",
  "gene_symbol": "CLVS2",
  "term_label": "endosome",
  "gene_name": "Clavesin-2",
  "gene": "UniProtKB:Q5SYC1"
}